membrane raft distribution [GO:0031580] (biological process) Sources: GOC:mah Also known as: lipid raft distribution Relationships: is a type of GO:0031579; is a type of membrane raft localization [GO:0051665] Definition: The process that establishes the spatial arrangement of membrane rafts within a cellular membrane. Subtypes: membrane raft polarization [GO:0001766], plasma membrane raft distribution [GO:0044855]